{
  "term_id": "GO:0000978",
  "gene_name": "Homeobox protein Hox-B2",
  "gene_symbol": "HOXB2",
  "term_label": "RNA polymerase II cis-regulatory region sequence-specific DNA binding",
  "gene": "UniProtKB:P14652"
}